{
  "gene_symbol": "EFCAB14",
  "gene_name": "EF-hand calcium-binding domain-containing protein 14",
  "term_label": "Unknown molecular function",
  "gene": "UniProtKB:O75071",
  "term_id": "UNKNOWN:0001"
}